positive regulation of protein targeting to vacuole involved in autophagy [GO:1904053] (biological process) Definition: Any process that activates or increases the frequency, rate or extent of protein targeting to vacuole involved in autophagy. References: PMID:22020285 Sources: GOC:PARL, GOC:TermGenie, GOC:pad, GO_REF:0000058 Also known as: up regulation of protein targeting to vacuole involved in autophagy, up-regulation of protein targeting to vacuole involved in autophagy, upregulation of protein targeting to vacuole involved in autophagy, activation of protein targeting to vacuole involved in autophagy Note: An example of this is SMURF1 in human (UniProt symbol Q9HCE7) in PMID:22020285 (inferred from mutant phenotype). Relationships: is a type of GO:0090316; is a type of positive regulation of vacuolar transport [GO:1903337]; is a type of regulation of protein targeting to vacuole involved in autophagy [GO:1904051]; positively regulates protein targeting to vacuole involved in autophagy [GO:0071211]